{
  "term_id": "GO:0070971",
  "gene_name": "Protein transport protein Sec31B",
  "gene_symbol": "SEC31B",
  "term_label": "endoplasmic reticulum exit site",
  "gene": "UniProtKB:Q9NQW1"
}